{
  "gene": "UniProtKB:O75155",
  "term_id": "GO:0005634",
  "gene_name": "Cullin-associated NEDD8-dissociated protein 2",
  "gene_symbol": "CAND2",
  "term_label": "nucleus"
}